{
  "gene": "UniProtKB:P01889",
  "term_label": "immune response",
  "term_id": "GO:0006955",
  "gene_symbol": "HLA-B",
  "gene_name": "HLA class I histocompatibility antigen, B alpha chain"
}